microtubule anchoring at cell cortex of cell tip [GO:0106007] (biological process) Relationships: is a type of GO:0034453 Definition: Any process in which a microtubule is maintained in a specific location at the cell tip by attachment to the cell cortex. References: PMID:25736293 Sources: GOC:mah